{
  "term_label": "Unknown biological process",
  "gene_name": "Uncharacterized protein",
  "gene_symbol": "A0A8I5KYW3",
  "gene": "UniProtKB:A0A8I5KYW3",
  "term_id": "UNKNOWN:0002"
}